{
  "gene_symbol": "SEPTIN11",
  "term_id": "GO:0003924",
  "gene": "UniProtKB:Q9NVA2",
  "gene_name": "Septin-11",
  "term_label": "GTPase activity"
}